positive regulation of canonical NF-kappaB signal transduction [GO:0043123] (biological process) Also known as: activation of I-kappaB kinase/NF-kappaB cascade, positive regulation of I-kappaB kinase/NF-kappaB cascade, positive regulation of I-kappaB kinase/NF-kappaB signaling, up regulation of I-kappaB kinase/NF-kappaB cascade, up-regulation of I-kappaB kinase/NF-kappaB cascade, upregulation of I-kappaB kinase/NF-kappaB cascade, stimulation of I-kappaB kinase/NF-kappaB cascade Relationships: is a type of GO:0043122; is a type of positive regulation of intracellular signal transduction [GO:1902533]; positively regulates GO:0007249 Sources: GOC:jl Definition: Any process that activates or increases the frequency, rate or extent of a canonical NF-kappaB signaling cascade.